negative regulation of glucocorticoid biosynthetic process [GO:0031947] (biological process) Definition: Any process that stops, prevents, or reduces the frequency, rate or extent of the chemical reactions and pathways resulting in the formation of glucocorticoids. Sources: GOC:mah Also known as: down regulation of glucocorticoid biosynthetic process, down-regulation of glucocorticoid biosynthetic process, downregulation of glucocorticoid biosynthetic process, inhibition of glucocorticoid biosynthetic process Relationships: is a type of regulation of glucocorticoid biosynthetic process [GO:0031946]; is a type of negative regulation of steroid hormone biosynthetic process [GO:0090032]; negatively regulates glucocorticoid biosynthetic process [GO:0006704] Subtypes: negative regulation of cortisol biosynthetic process [GO:2000065]